{
  "gene_symbol": "AKR1C1",
  "gene_name": "Aldo-keto reductase family 1 member C1",
  "gene": "UniProtKB:Q04828",
  "term_label": "doxorubicin metabolic process",
  "term_id": "GO:0044598"
}